import into nucleus [GO:0051170] (biological process) Definition: The directed movement of substances into the nucleus. Relationships: is a type of nucleocytoplasmic transport [GO:0006913] Also known as: nuclear import, nuclear translocation Sources: GOC:ai Subtypes: RNA import into nucleus [GO:0006404], protein import into nucleus [GO:0006606], proteasome core complex import into nucleus [GO:1990236]